vasoconstriction of artery involved in carotid body chemoreceptor response to lowering of systemic arterial blood pressure [GO:0003042] (biological process) Relationships: is a type of vasoconstriction of artery involved in chemoreceptor response to lowering of systemic arterial blood pressure [GO:0002012]; is part of GO:0003027 Also known as: vasoconstriction of artery during carotid body chemoreceptor response to lowering of systemic arterial blood pressure Definition: A process that is triggered by carotid body-vasomotor excitation and results in a decrease in the diameter of an artery during the chemoreceptor response to decreased blood pressure. Sources: ISBN:0323031951